cell differentiation involved in kidney development [GO:0061005] (biological process) Subtypes: epithelial cell differentiation involved in kidney development [GO:0035850], cell differentiation involved in pronephros development [GO:0039014], cell differentiation involved in mesonephros development [GO:0061208], GO:0072007, mesenchymal stem cell differentiation involved in nephron morphogenesis [GO:0072037], juxtaglomerulus cell differentiation [GO:0072052], proximal convoluted tubule segment 1 cell differentiation [GO:0072062], DCT cell differentiation [GO:0072069], kidney interstitial fibroblast differentiation [GO:0072071], mesenchymal cell differentiation involved in kidney development [GO:0072161], renal vesicle progenitor cell differentiation [GO:0072184], GO:0072195, cell differentiation involved in metanephros development [GO:0072202] Definition: The process in which relatively unspecialized cells acquire specialized structural and/or functional features that characterize the cells of the kidney as it progresses from its formation to the mature state. Relationships: is a type of cell differentiation [GO:0030154]; is part of kidney development [GO:0001822] Sources: GOC:mtg_kidney_jan10